{
  "gene_symbol": "ZNF350",
  "gene": "UniProtKB:Q9GZX5",
  "gene_name": "Zinc finger protein 350",
  "term_label": "regulation of transcription by RNA polymerase II",
  "term_id": "GO:0006357"
}